{
  "term_id": "GO:0005615",
  "term_label": "extracellular space",
  "gene_name": "Resistin-like beta",
  "gene": "UniProtKB:Q9BQ08",
  "gene_symbol": "RETNLB"
}